{
  "gene_name": "T-lymphocyte activation antigen CD86",
  "gene": "UniProtKB:P42081",
  "gene_symbol": "CD86",
  "term_label": "negative regulation of T cell proliferation",
  "term_id": "GO:0042130"
}